{
  "term_label": "signaling receptor binding",
  "gene": "UniProtKB:O60687",
  "gene_symbol": "SRPX2",
  "term_id": "GO:0005102",
  "gene_name": "Sushi repeat-containing protein SRPX2"
}